endocardial cushion morphogenesis [GO:0003203] (biological process) Sources: GOC:mtg_heart Relationships: is a type of GO:0072132; is part of heart morphogenesis [GO:0003007]; is part of endocardial cushion development [GO:0003197] Definition: The process in which the anatomical structure of the endocardial cushion is generated and organized. The endocardial cushion is a specialized region of mesenchymal cells that will give rise to the heart septa and valves. Subtypes: superior endocardial cushion morphogenesis [GO:1905316], inferior endocardial cushion morphogenesis [GO:1905317]